{
  "term_label": "establishment or maintenance of cell polarity",
  "term_id": "GO:0007163",
  "gene_name": "Rho-related BTB domain-containing protein 2",
  "gene_symbol": "RHOBTB2",
  "gene": "UniProtKB:Q9BYZ6"
}